regulation of toll-like receptor 8 signaling pathway [GO:0034159] (biological process) Relationships: is a type of GO:0039531; regulates GO:0034158 Definition: Any process that modulates the frequency, rate, or extent of toll-like receptor 8 signaling pathway. References: PMID:16551253, PMID:17328678 Sources: GOC:add Subtypes: negative regulation of toll-like receptor 8 signaling pathway [GO:0034160], positive regulation of toll-like receptor 8 signaling pathway [GO:0034161] Also known as: regulation of TLR8 signaling pathway, regulation of toll-like receptor 8 signalling pathway